{
  "term_id": "GO:0010521",
  "gene_name": "CST complex subunit TEN1",
  "term_label": "telomerase inhibitor activity",
  "gene_symbol": "TEN1",
  "gene": "UniProtKB:Q86WV5"
}